ornithine N5-monooxygenase activity [GO:0031172] (MF) Definition: Catalysis of the reaction: L-ornithine + O2 + H+ = N5-hydroxy-L-ornithine + H2O. Relationships: is a type of monooxygenase activity [GO:0004497] Also known as: L-ornithine 5-monooxygenase activity References: PMID:12828635 Sources: MetaCyc:RXN-11128